double-strand break repair involved in meiotic recombination [GO:1990918] (biological process) Definition: The repair of double-strand breaks in DNA via homologous and nonhomologous mechanisms to reform a continuous DNA helix that contributes to reciprocal meiotic recombination. References: PMID:15238514 Sources: GOC:mah Relationships: is a type of double-strand break repair [GO:0006302]; is a type of meiotic cell cycle process [GO:1903046]; is part of reciprocal meiotic recombination [GO:0007131]